aflatoxin reductase (coenzyme F420) activity [GO:0052807] (molecular function) Definition: Catalysis of the reaction: aflatoxin + 1,5-dihydrocoenzyme F420 = aflatoxin with reduced furanocoumarin moiety + coenzyme F420. 1,5-dihydrocoenzyme F420 is also known as reduced coenzyme F420. Also known as: aflatoxin:coenzyme F420 oxidoreductase activity, aflatoxin:reduced coenzyme F420 reductase activity, coenzyme F420-aflatoxin reductase activity, coenzyme F420-dependent aflatoxin reductase activity Relationships: is a type of GO:0016667; is part of GO:0046223 References: PMID:20807200 Sources: GOC:mengo_curators